regulation of translation involved in cellular response to UV [GO:1904803] (biological process) Definition: Any regulation of translation that is involved in cellular response to UV. Also known as: regulation of protein anabolism involved in cellular response to UV, regulation of protein biosynthesis involved in cellular response to UV, regulation of protein formation involved in cellular response to UV, regulation of protein synthesis involved in cellular response to UV, regulation of translation involved in cellular response to UV light stimulus, regulation of translation involved in cellular response to UV radiation stimulus, regulation of translation involved in cellular response to ultraviolet light stimulus, regulation of translation involved in cellular response to ultraviolet radiation stimulus Relationships: is a type of regulation of translation [GO:0006417]; BFO_0000050 cellular response to UV [GO:0034644] References: PMID:17369398 Sources: GOC:TermGenie, GO_REF:0000060